{
  "gene": "UniProtKB:Q96N22",
  "term_label": "DNA-binding transcription factor activity, RNA polymerase II-specific",
  "gene_symbol": "ZNF681",
  "gene_name": "Zinc finger protein 681",
  "term_id": "GO:0000981"
}